{
  "term_id": "GO:0002767",
  "gene": "UniProtKB:Q9HCN6",
  "term_label": "immune response-inhibiting cell surface receptor signaling pathway",
  "gene_name": "Platelet glycoprotein VI",
  "gene_symbol": "GP6"
}